{
  "gene_name": "Ras-related protein Rab-9B",
  "term_id": "GO:0045335",
  "term_label": "phagocytic vesicle",
  "gene_symbol": "RAB9B",
  "gene": "UniProtKB:Q9NP90"
}